egg deposition [GO:0160027] (biological process) Definition: The multicellular organismal reproductive process that results in the movement of an egg from within an organism into the external environment. References: PMID:18050396, PMID:31164023 Relationships: is a type of multicellular organismal reproductive process [GO:0048609]